{
  "gene_symbol": "GFY",
  "gene_name": "Golgi-associated olfactory signaling regulator",
  "gene": "UniProtKB:I3L273",
  "term_label": "Unknown molecular function",
  "term_id": "UNKNOWN:0001"
}